{
  "gene_name": "Putative testis-specific Y-encoded-like protein 3",
  "gene_symbol": "TSPY26P",
  "gene": "UniProtKB:Q9H489",
  "term_label": "nucleus",
  "term_id": "GO:0005634"
}